{
  "gene_symbol": "KIF1C",
  "gene": "UniProtKB:O43896",
  "term_label": "cytoplasm",
  "gene_name": "Kinesin-like protein KIF1C",
  "term_id": "GO:0005737"
}